difructose-anhydride synthase activity [GO:0047853] (molecular function) Definition: Catalysis of the reaction: H2O + bis-D-fructose 2',1:2,1'-dianhydride = inulobiose. Sources: MetaCyc:DIFRUCTOSE-ANHYDRIDE-SYNTHASE-RXN, RHEA:15041 Also known as: bis-D-fructose 2',1:2,1'-dianhydride fructohydrolase activity, inulobiose hydrolase activity Relationships: is a type of hydrolase activity, hydrolyzing O-glycosyl compounds [GO:0004553]